N-acyl-D-aspartate deacylase activity [GO:0047422] (molecular function) Definition: Catalysis of the reaction: N-acyl-D-aspartate + H2O = D-aspartate + a carboxylate. Relationships: is a type of GO:0016811 Also known as: N-acyl-D-aspartate amidohydrolase activity Sources: EC:3.5.1.83, RHEA:18285